{
  "term_label": "Unknown cellular component",
  "gene_symbol": "TMEM176A",
  "term_id": "UNKNOWN:0003",
  "gene_name": "Transmembrane protein 176A",
  "gene": "UniProtKB:Q96HP8"
}